{
  "term_label": "acid-amino acid ligase activity",
  "term_id": "GO:0016881",
  "gene_name": "GH3 domain-containing protein",
  "gene_symbol": "GHDC",
  "gene": "UniProtKB:Q8N2G8"
}